3'-tyrosyl-DNA phosphodiesterase activity [GO:0017005] (molecular function) Definition: Catalysis of the hydrolysis of 3'-phosphotyrosyl groups formed as covalent intermediates (in DNA backbone breakage) between DNA topoisomerase I and DNA. References: PMID:10521354, PMID:16751265 Relationships: is_a tyrosyl-DNA phosphodiesterase activity [GO:0070259] Note: See also the molecular function term 'DNA topoisomerase type I activity ; GO:0003917'.